{
  "gene_symbol": "TRAV40",
  "gene": "UniProtKB:A0A0B4J280",
  "term_label": "adaptive immune response",
  "term_id": "GO:0002250",
  "gene_name": "T cell receptor alpha variable 40"
}